{
  "term_label": "regulation of pyruvate decarboxylation to acetyl-CoA",
  "term_id": "GO:0010510",
  "gene": "UniProtKB:Q16654",
  "gene_symbol": "PDK4",
  "gene_name": "[Pyruvate dehydrogenase (acetyl-transferring)] kinase isozyme 4, mitochondrial"
}